{
  "gene_name": "Cytoplasmic FMR1-interacting protein 1",
  "term_id": "GO:0031209",
  "gene": "UniProtKB:Q7L576",
  "term_label": "SCAR complex",
  "gene_symbol": "CYFIP1"
}